{
  "term_label": "protein import into nucleus",
  "gene_name": "Protein FAM53C",
  "gene": "UniProtKB:Q9NYF3",
  "gene_symbol": "FAM53C",
  "term_id": "GO:0006606"
}